{
  "gene_symbol": "DOK2",
  "gene_name": "Docking protein 2",
  "term_id": "UNKNOWN:0003",
  "gene": "UniProtKB:O60496",
  "term_label": "Unknown cellular component"
}